carbon dioxide transport [GO:0015670] (biological process) Definition: The directed movement of carbon dioxide (CO2) into, out of or within a cell, or between cells, by means of some agent such as a transporter or pore. Relationships: is a type of GO:0015669; is a type of one-carbon compound transport [GO:0019755] Subtypes: carbon dioxide transmembrane transport [GO:0035378] Sources: GOC:ai